{
  "gene": "UniProtKB:P51828",
  "gene_name": "Adenylate cyclase type 7",
  "term_label": "adenylate cyclase-activating G protein-coupled receptor signaling pathway",
  "term_id": "GO:0007189",
  "gene_symbol": "ADCY7"
}